activation of mitotic cell cycle spindle assembly checkpoint [GO:0090268] (biological process) Relationships: is a type of positive regulation of mitotic cell cycle spindle assembly checkpoint [GO:0090267] Definition: Any process that starts the inactive process of a mitotic cell cycle spindle assembly checkpoint. Sources: GOC:mah, GOC:vw